positive regulation of glycerol transport [GO:0090372] (biological process) Definition: Any process that increases the rate, frequency, or extent of the directed movement of glycerol into, out of or within a cell, or between cells, by means of some agent such as a transporter or pore. Relationships: is a type of GO:0034764; is a type of regulation of glycerol transport [GO:0090371]; positively regulates GO:0015793 Sources: GOC:dph, GOC:jh, GOC:tb